alkane 1-monooxygenase activity [GO:0018685] (molecular function) Sources: RHEA:19341 Relationships: is a type of oxidoreductase activity, acting on paired donors, with incorporation or reduction of molecular oxygen, reduced iron-sulfur protein as one donor, and incorporation of one atom of oxygen [GO:0016713] Definition: Catalysis of the reaction: octane + reduced rubredoxin + O2 = 1-octanol + oxidized rubredoxin + H2O. Also known as: alkane 1-hydroxylase activity, 1-hydroxylase activity, alkane hydroxylase activity, alkane monooxygenase activity, alkane,reduced-rubredoxin:oxygen 1-oxidoreductase activity